{
  "gene_symbol": "C3orf18",
  "term_id": "UNKNOWN:0002",
  "term_label": "Unknown biological process",
  "gene_name": "Uncharacterized protein C3orf18",
  "gene": "UniProtKB:Q9UK00"
}